reservosome matrix [GO:0106125] (cellular component) Definition: A matrix composed of planar membranes, vesicles and lipid inclusions within the reservosome. References: PMID:12204365, PMID:15521631, PMID:18452191, PMID:19288526, PMID:21818313, PMID:22425988 Sources: GOC:ach Relationships: is a type of cellular anatomical structure [GO:0110165]; is part of reservosome [GO:0106123]